{
  "gene_name": "Serine protease inhibitor Kazal-type 2",
  "term_id": "GO:0007286",
  "gene": "UniProtKB:P20155",
  "gene_symbol": "SPINK2",
  "term_label": "spermatid development"
}